{
  "term_id": "GO:0008284",
  "gene_name": "Regenerating islet-derived protein 3-gamma",
  "term_label": "positive regulation of cell population proliferation",
  "gene": "UniProtKB:Q6UW15",
  "gene_symbol": "REG3G"
}